{
  "gene": "UniProtKB:Q8ND71",
  "gene_name": "GTPase IMAP family member 8",
  "gene_symbol": "GIMAP8",
  "term_label": "endoplasmic reticulum",
  "term_id": "GO:0005783"
}